negative regulation of protein localization to kinetochore [GO:1905341] (biological process) Definition: Any process that stops, prevents or reduces the frequency, rate or extent of protein localization to kinetochore. References: PMID:22581055 Sources: GOC:TermGenie, GO_REF:0000058 Also known as: down regulation of protein localisation to kinetochore, down regulation of protein localization to kinetochore, down-regulation of protein localisation to kinetochore, down-regulation of protein localization to kinetochore, downregulation of protein localisation to kinetochore, downregulation of protein localization to kinetochore, negative regulation of protein localisation to kinetochore, down regulation of condensin localization to kinetochore, down-regulation of condensin localization to kinetochore, downregulation of condensin localization to kinetochore, inhibition of condensin localization to kinetochore, inhibition of protein localisation to kinetochore, inhibition of protein localization to kinetochore, negative regulation of condensin localization to kinetochore Note: Q9H211 in Human in PMID:22581055 Relationships: is a type of negative regulation of protein localization [GO:1903828]; is a type of regulation of protein localization to kinetochore [GO:1905340]; negatively regulates GO:0034501